{
  "gene": "UniProtKB:P09210",
  "term_label": "cytosol",
  "term_id": "GO:0005829",
  "gene_name": "Glutathione S-transferase A2",
  "gene_symbol": "GSTA2"
}